6-amino-6-deoxyfutalosine hydrolase activity [GO:0102246] (molecular function) Sources: EC:3.2.2.30, GOC:pz Definition: Catalysis of the reaction: aminodeoxyfutalosinate + H2O = dehypoxanthine futalosine + adenine. Relationships: is a type of hydrolase activity, hydrolyzing N-glycosyl compounds [GO:0016799]